{
  "gene_symbol": "NACAD",
  "gene": "UniProtKB:O15069",
  "term_label": "cytoplasm",
  "gene_name": "NAC-alpha domain-containing protein 1",
  "term_id": "GO:0005737"
}